{
  "gene_symbol": "NYNRIN",
  "term_label": "cytoplasmic ribonucleoprotein granule",
  "gene": "UniProtKB:Q9P2P1",
  "term_id": "GO:0036464",
  "gene_name": "Protein NYNRIN"
}